SAGA complex [GO:0000124] (cellular component) Definition: A SAGA-type histone acetyltransferase complex that deubiquitinates H2A and/or H2B. This complex is organized into several functional submodules: a structural core including the activator binding module and consisting of ADA1 or a homolog, members of the SPT and TAF protein families as well as promotor recruitment factor TRRAP/TRA1, a histone acetyltransferase (HAT) module consisting of GCN5/KAT2A or PCAF/KAT2B, ADA2, ADA3/NGG1, and SGF29 or homologues thereof, a histone deubiquitinase (DUB) module consisting of ATXN7/SGF73, ATXN7L3/SGF11, ENY2/SUS1 and USP22/UBP8 or homologues thereof, and in some taxa a splicing module consisting of SF3B3 and SF3B5 or homologues thereof (not in fungi). In budding yeast also contains Spt8 which distinguishes it from SAGA-like (SLIK) complex (GO:0046695). References: PMID:10637607, PMID:17337012, PMID:19056896, PMID:20838651, PMID:33004486 Also known as: Spt-Ada-Gcn5-acetyltransferase complex, PCAF complex, PCAF histone acetylase-associated complex, SPT3-TAF9-PCAF acetylase complex, SPT3-TAF9-GCN5 acetylase complex, STAGA coactivator complex, STAGA complex Relationships: is_a SAGA-type complex [GO:0070461]; is a type of peptidase complex [GO:1905368]; has part GO:0071819